{
  "term_id": "UNKNOWN:0001",
  "gene_name": "Tectonic-1",
  "term_label": "Unknown molecular function",
  "gene_symbol": "TCTN1",
  "gene": "UniProtKB:Q2MV58"
}